{
  "gene": "UniProtKB:A6NI73",
  "gene_symbol": "LILRA5",
  "term_label": "cytokine-mediated signaling pathway",
  "term_id": "GO:0019221",
  "gene_name": "Leukocyte immunoglobulin-like receptor subfamily A member 5"
}